{
  "term_label": "receptor internalization",
  "gene_symbol": "RAMP3",
  "gene_name": "Receptor activity-modifying protein 3",
  "term_id": "GO:0031623",
  "gene": "UniProtKB:O60896"
}